{
  "gene_symbol": "NKAIN4",
  "term_label": "Unknown molecular function",
  "gene": "UniProtKB:Q8IVV8",
  "gene_name": "Sodium_potassium-transporting ATPase subunit beta-1-interacting protein 4",
  "term_id": "UNKNOWN:0001"
}